{
  "gene_symbol": "ENPP3",
  "term_id": "UNKNOWN:0003",
  "gene_name": "Ectonucleotide pyrophosphatase_phosphodiesterase family member 3",
  "term_label": "Unknown cellular component",
  "gene": "UniProtKB:O14638"
}